regulation of mitochondrial outer membrane permeabilization involved in apoptotic signaling pathway [GO:1901028] (biological process) Subtypes: negative regulation of mitochondrial outer membrane permeabilization involved in apoptotic signaling pathway [GO:1901029], positive regulation of mitochondrial outer membrane permeabilization involved in apoptotic signaling pathway [GO:1901030] Definition: Any process that modulates the frequency, rate or extent of mitochondrial outer membrane permeabilization involved in apoptotic signaling pathway. Also known as: regulation of mitochondrial outer membrane permeabilization, regulation of MOMP Sources: GOC:BHF, GOC:TermGenie, GOC:mtg_apoptosis Relationships: is_a regulation of mitochondrion organization [GO:0010821]; is a type of regulation of mitochondrial membrane permeability [GO:0046902]; is a type of regulation of transport [GO:0051049]; regulates mitochondrial outer membrane permeabilization [GO:0097345]